{
  "gene_symbol": "SLC27A1",
  "term_id": "GO:0090434",
  "gene_name": "Long-chain fatty acid transport protein 1",
  "term_label": "oleoyl-CoA ligase activity",
  "gene": "UniProtKB:Q6PCB7"
}